{
  "term_id": "GO:0022627",
  "gene_symbol": "RPS5",
  "term_label": "cytosolic small ribosomal subunit",
  "gene": "UniProtKB:P46782",
  "gene_name": "Small ribosomal subunit protein uS7"
}